{
  "gene_symbol": "TNFRSF18",
  "term_label": "external side of plasma membrane",
  "gene": "UniProtKB:Q9Y5U5",
  "term_id": "GO:0009897",
  "gene_name": "Tumor necrosis factor receptor superfamily member 18"
}